positive regulation of nuclear receptor-mediated glucocorticoid signaling pathway [GO:2000324] (biological process) Sources: GOC:BHF Also known as: positive regulation of glucocorticoid receptor signaling pathway, positive regulation of glucocorticoid receptor signalling pathway Relationships: is a type of positive regulation of intracellular steroid hormone receptor signaling pathway [GO:0033145]; is a type of regulation of nuclear receptor-mediated glucocorticoid signaling pathway [GO:2000322]; positively regulates nuclear receptor-mediated glucocorticoid signaling pathway [GO:0042921] Definition: Any process that activates or increases the frequency, rate or extent of nuclear receptor-mediated glucocorticoid signaling pathway.